regulation of macrophage migration inhibitory factor signaling pathway [GO:2000446] (biological process) Definition: Any process that modulates the frequency, rate or extent of macrophage migration inhibitory factor signaling pathway. Sources: GOC:obol Relationships: is a type of regulation of cytokine-mediated signaling pathway [GO:0001959]; regulates macrophage migration inhibitory factor signaling pathway [GO:0035691] Subtypes: negative regulation of macrophage migration inhibitory factor signaling pathway [GO:2000447], positive regulation of macrophage migration inhibitory factor signaling pathway [GO:2000448] Also known as: regulation of MIF signaling pathway, regulation of macrophage migration inhibitory factor signalling pathway